chloroplast rRNA processing [GO:1901259] (biological process) Definition: Any rRNA processing that takes place in chloroplast. Sources: GOC:TermGenie Relationships: is a type of rRNA processing [GO:0006364]; occurs in chloroplast [GO:0009507]